{
  "term_id": "UNKNOWN:0002",
  "gene_symbol": "TRIM8",
  "term_label": "Unknown biological process",
  "gene": "UniProtKB:Q9BZR9",
  "gene_name": "E3 ubiquitin-protein ligase TRIM8"
}